aspulvinone dimethylallyltransferase activity [GO:0047691] (molecular function) Also known as: dimethylallyl pyrophosphate:aspulvinone dimethylallyltransferase activity, dimethylallyl-diphosphate:aspulvinone-E dimethylallyltransferase activity Sources: EC:2.5.1.35, RHEA:13809 Relationships: is a type of transferase activity, transferring alkyl or aryl (other than methyl) groups [GO:0016765] Definition: Catalysis of the reaction: aspulvinone E + 2 dimethylallyl diphosphate = aspulvinone H + 2 diphosphate.